{
  "gene": "UniProtKB:Q9NTU7",
  "gene_symbol": "CBLN4",
  "gene_name": "Cerebellin-4",
  "term_label": "synapse",
  "term_id": "GO:0045202"
}